growth involved in heart morphogenesis [GO:0003241] (biological process) Relationships: is a type of developmental growth involved in morphogenesis [GO:0060560]; is part of heart morphogenesis [GO:0003007]; BFO_0000050 heart growth [GO:0060419] Subtypes: cardiac chamber ballooning [GO:0003242], GO:0003243, radial growth involved in right ventricle morphogenesis [GO:0003244], cardiac muscle tissue growth involved in heart morphogenesis [GO:0003245], embryonic cardiac muscle cell growth involved in heart morphogenesis [GO:0003246], post-embryonic cardiac muscle cell growth involved in heart morphogenesis [GO:0003247] Definition: Developmental growth that contributes to the shaping of the heart. Sources: GOC:mtg_heart